immunoglobulin complex [GO:0019814] (CC) Also known as: antibody Sources: GOC:add, GOC:jl, ISBN:0781765196 Definition: A protein complex that in its canonical form is composed of two identical immunoglobulin heavy chains and two identical immunoglobulin light chains, held together by disulfide bonds and sometimes complexed with additional proteins. An immunoglobulin complex may be embedded in the plasma membrane or present in the extracellular space, in mucosal areas or other tissues, or circulating in the blood or lymph. Relationships: is a type of GO:0032991 Subtypes: GO:0019815, immunoglobulin complex, circulating [GO:0042571], GO:0071735, IgD immunoglobulin complex [GO:0071738], GO:0071742, GO:0071745, IgM immunoglobulin complex [GO:0071753], IgW immunoglobulin complex [GO:0071758], IgX immunoglobulin complex [GO:0071759], GO:0071760, IgZ immunoglobulin complex [GO:0071761], heavy chain immunoglobulin complex [GO:0071762] Note: Note that an immunoglobulin complex has the function of antigen binding if a suitable antigen is available.